{
  "gene_symbol": "ZNF8",
  "gene_name": "Zinc finger protein 8",
  "gene": "UniProtKB:P17098",
  "term_id": "GO:0000981",
  "term_label": "DNA-binding transcription factor activity, RNA polymerase II-specific"
}